{
  "term_label": "L-glutamate import across plasma membrane",
  "gene_symbol": "SLC1A2",
  "gene": "UniProtKB:P43004",
  "gene_name": "Excitatory amino acid transporter 2",
  "term_id": "GO:0098712"
}